negative regulation of neural retina development [GO:0061076] (biological process) Definition: Any process that decreases the rate, frequency, or extent of neural retina development, the progression of the neural retina over time from its initial formation to the mature structure. The neural retina is the part of the retina that contains neurons and photoreceptor cells. Sources: GOC:dph Relationships: is a type of regulation of neural retina development [GO:0061074]; is a type of negative regulation of retina development in camera-type eye [GO:1902867]; negatively regulates neural retina development [GO:0003407]